{
  "term_label": "establishment of skin barrier",
  "gene_symbol": "FLG2",
  "gene": "UniProtKB:Q5D862",
  "gene_name": "Filaggrin-2",
  "term_id": "GO:0061436"
}